{
  "gene_name": "Protocadherin-8",
  "gene": "UniProtKB:O95206",
  "gene_symbol": "PCDH8",
  "term_id": "GO:0045202",
  "term_label": "synapse"
}